{
  "gene": "UniProtKB:Q9H2U6",
  "gene_name": "Putative uncharacterized protein encoded by LINC00597",
  "gene_symbol": "LINC00597",
  "term_label": "Unknown biological process",
  "term_id": "UNKNOWN:0002"
}